{
  "gene": "UniProtKB:Q9H3H9",
  "gene_symbol": "TCEAL2",
  "term_id": "UNKNOWN:0003",
  "term_label": "Unknown cellular component",
  "gene_name": "Transcription elongation factor A protein-like 2"
}